{
  "term_id": "UNKNOWN:0003",
  "gene_name": "Zinc finger protein 592",
  "gene": "UniProtKB:Q92610",
  "term_label": "Unknown cellular component",
  "gene_symbol": "ZNF592"
}